{
  "term_label": "Unknown biological process",
  "gene": "UniProtKB:P59551",
  "gene_symbol": "TAS2R60",
  "gene_name": "Taste receptor type 2 member 60",
  "term_id": "UNKNOWN:0002"
}